{
  "gene_symbol": "SPDYE15",
  "gene": "UniProtKB:P0DUD4",
  "term_label": "Unknown biological process",
  "term_id": "UNKNOWN:0002",
  "gene_name": "Putative speedy protein E15"
}